{
  "gene_symbol": "SCARF1",
  "gene": "UniProtKB:Q14162",
  "term_id": "GO:0016322",
  "term_label": "neuron remodeling",
  "gene_name": "Scavenger receptor class F member 1"
}